{
  "gene": "UniProtKB:Q86YW5",
  "term_id": "GO:0004888",
  "gene_name": "Trem-like transcript 1 protein",
  "term_label": "transmembrane signaling receptor activity",
  "gene_symbol": "TREML1"
}